aorta development [GO:0035904] (biological process) Definition: The progression of the aorta over time, from its initial formation to the mature structure. An aorta is an artery that carries blood from the heart to other parts of the body. Sources: GOC:bf, GOC:dgh, MA:0000062, UBERON:0000947, Wikipedia:Aorta Subtypes: GO:0035907, ventral aorta development [GO:0035908] Relationships: is a type of artery development [GO:0060840]